{
  "gene": "UniProtKB:Q96PQ7",
  "term_label": "proteasome-mediated ubiquitin-dependent protein catabolic process",
  "gene_symbol": "KLHL5",
  "term_id": "GO:0043161",
  "gene_name": "Kelch-like protein 5"
}